{
  "term_label": "Unknown biological process",
  "term_id": "UNKNOWN:0002",
  "gene": "UniProtKB:Q0IIN9",
  "gene_symbol": "ZNF252P-AS1",
  "gene_name": "Putative uncharacterized protein ZNF252P-AS1"
}